transcription-coupled nucleotide-excision repair [GO:0006283] (biological process) Also known as: TC-NER, transcription-coupled NER, transcription-coupled repair, TCR Definition: The nucleotide-excision repair process that carries out preferential repair of DNA lesions on the actively transcribed strand of the DNA duplex. In addition, the transcription-coupled nucleotide-excision repair pathway is required for the recognition and repair of a small subset of lesions that are not recognized by the global genome nucleotide excision repair pathway. References: PMID:10197977, PMID:11900249 Relationships: is a type of nucleotide-excision repair [GO:0006289] Regulation: regulated by regulation of transcription-coupled nucleotide-excision repair [GO:0090262]